neurotrophin TRKC receptor binding [GO:0005170] (MF) Sources: GOC:ai Also known as: neurotrophin TRKC receptor ligand Definition: Binding to a neurotrophin TRKC receptor. Relationships: is a type of GO:0005167